protein histidine pros-kinase activity [GO:0008256] (molecular function) Definition: Catalysis of the reaction: ATP + protein L-histidine = ADP + protein N(pi)-phospho-L-histidine. Sources: EC:2.7.13.1 Also known as: ATP:protein-L-histidine Npi-phosphotransferase activity, protein-histidine pros-kinase activity, ATP:protein-L-histidine N-pros-phosphotransferase activity Relationships: is a type of protein histidine kinase activity [GO:0004673]